hexitol dehydrogenase activity [GO:0031320] (molecular function) Relationships: is_a oxidoreductase activity, acting on CH-OH group of donors [GO:0016614] Sources: GOC:mah Subtypes: mannitol dehydrogenase activity [GO:0046029], D-xylulose reductase activity [GO:0046526], galactitol 2-dehydrogenase activity [GO:0047713], D-iditol 2-dehydrogenase activity [GO:0047824] Definition: Catalysis of the reaction: hexitol + acceptor = hexose + reduced acceptor.